{
  "term_label": "nucleus",
  "gene_name": "Protein CBFA2T3",
  "term_id": "GO:0005634",
  "gene": "UniProtKB:O75081",
  "gene_symbol": "CBFA2T3"
}